{
  "term_id": "UNKNOWN:0003",
  "gene": "UniProtKB:A0A075B6W6",
  "gene_name": "T cell receptor alpha joining 27 (Fragment)",
  "gene_symbol": "TRAJ27",
  "term_label": "Unknown cellular component"
}